{
  "gene": "UniProtKB:Q86YD7",
  "gene_name": "Protein FAM90A1",
  "term_label": "Unknown cellular component",
  "gene_symbol": "FAM90A1",
  "term_id": "UNKNOWN:0003"
}